{
  "term_label": "Unknown molecular function",
  "gene_symbol": "NGRN",
  "gene": "UniProtKB:Q9NPE2",
  "term_id": "UNKNOWN:0001",
  "gene_name": "Neugrin"
}